{
  "gene": "UniProtKB:P50613",
  "term_label": "cytoplasm",
  "gene_name": "Cyclin-dependent kinase 7",
  "gene_symbol": "CDK7",
  "term_id": "GO:0005737"
}